{
  "gene": "UniProtKB:O75602",
  "term_label": "sperm principal piece",
  "gene_symbol": "SPAG6",
  "term_id": "GO:0097228",
  "gene_name": "Sperm-associated antigen 6"
}